{
  "term_label": "intracellular calcium ion homeostasis",
  "gene": "UniProtKB:P20800",
  "gene_name": "Endothelin-2",
  "term_id": "GO:0006874",
  "gene_symbol": "EDN2"
}